initiation of movement involved in cerebral cortex radial glia guided migration [GO:0021806] (biological process) Definition: The initial stages of cell motility involved in the glial-mediated movement of cells in the developing cerebral cortex. References: PMID:12626695 Sources: GOC:cls, GOC:dgh, GOC:dph, GOC:jid, GO_REF:0000021 Also known as: initiation of movement involved in cerebral cortex glial-mediated radial migration Relationships: is_a cellular developmental process [GO:0048869]; BFO_0000050 ameboidal-type cell migration [GO:0001667]; is part of GO:0021814